{
  "gene_name": "T cell receptor delta variable 1",
  "gene_symbol": "TRDV1",
  "term_id": "UNKNOWN:0001",
  "term_label": "Unknown molecular function",
  "gene": "UniProtKB:A0A1B0GX56"
}